{
  "gene_name": "Lysine-specific demethylase hairless",
  "term_id": "GO:0003712",
  "gene": "UniProtKB:O43593",
  "term_label": "transcription coregulator activity",
  "gene_symbol": "HR"
}